{
  "gene_name": "Golgin subfamily A member 8J",
  "term_label": "cis-Golgi network",
  "gene_symbol": "GOLGA8J",
  "gene": "UniProtKB:A6NMD2",
  "term_id": "GO:0005801"
}